stem cell proliferation [GO:0072089] (biological process) Regulation: regulated by regulation of stem cell proliferation [GO:0072091]; negatively regulated by negative regulation of stem cell proliferation [GO:2000647]; positively regulated by positive regulation of stem cell proliferation [GO:2000648] Relationships: is a type of cell population proliferation [GO:0008283]; has part GO:0017145 Sources: GOC:mtg_kidney_jan10 Definition: The multiplication or reproduction of stem cells, resulting in the expansion of a stem cell population. A stem cell is a cell that retains the ability to divide and proliferate throughout life to provide progenitor cells that can differentiate into specialized cells. Subtypes: hematopoietic stem cell proliferation [GO:0071425], mesenchymal stem cell proliferation [GO:0097168]